mitotic morphogenesis checkpoint signaling [GO:0044879] (biological process) Also known as: morphogenesis checkpoint, septin checkpoint, signal transduction involved in morphogenesis checkpoint, signal transduction involved in septin checkpoint, signaling cascade involved in morphogenesis checkpoint, signaling cascade involved in septin checkpoint, signaling pathway involved in morphogenesis checkpoint, signaling pathway involved in septin checkpoint, signalling cascade involved in morphogenesis checkpoint, signalling cascade involved in septin checkpoint, signalling pathway involved in morphogenesis checkpoint, signalling pathway involved in septin checkpoint Relationships: is a type of mitotic cell cycle checkpoint signaling [GO:0007093] Definition: A signaling process that contributes to a mitotic cell cycle checkpoint which delays mitotic onset in response to perturbations that affect cell shape via the actin cytoskeleton, septin organization, small cell size, and/or the extent of membrane growth. Sources: GOC:jl, GOC:mtg_cell_cycle